{
  "term_label": "plasma membrane",
  "gene": "UniProtKB:Q9P296",
  "gene_name": "C5a anaphylatoxin chemotactic receptor 2",
  "gene_symbol": "C5AR2",
  "term_id": "GO:0005886"
}